{
  "gene": "UniProtKB:Q9BZV3",
  "term_id": "UNKNOWN:0003",
  "term_label": "Unknown cellular component",
  "gene_name": "Interphotoreceptor matrix proteoglycan 2",
  "gene_symbol": "IMPG2"
}